glycogen biosynthetic process via ADP-glucose [GO:0160250] (BP) Sources: MetaCyc:GLYCOGENSYNTH-PWY Definition: The chemical reactions and pathways resulting in the formation of glycogen, a polydisperse, highly branched glucan composed of chains of D-glucose residues, occurring through a ADP-glucose intermediate. Relationships: is a type of glycogen biosynthetic process [GO:0005978]